{
  "gene": "UniProtKB:P35638",
  "gene_name": "DNA damage-inducible transcript 3 protein",
  "gene_symbol": "DDIT3",
  "term_id": "GO:1990622",
  "term_label": "CHOP-ATF3 complex"
}